uridine-rich cytoplasmic polyadenylylation element binding [GO:0017131] (molecular function) Definition: Binding to a U-rich sequence in the 3'-end of nuclear-transcribed mRNAs; required for cytoplasmic polyadenylylation. Relationships: is a type of GO:0008187 Also known as: U-rich CPE binding, uridine-rich cytoplasmic polyadenylation element binding References: PMID:7954828 Sources: GOC:krc